{
  "gene_symbol": "HCN3",
  "term_label": "axon",
  "gene": "UniProtKB:Q9P1Z3",
  "gene_name": "Potassium_sodium hyperpolarization-activated cyclic nucleotide-gated channel 3",
  "term_id": "GO:0030424"
}